negative regulation of GDF15-GFRAL signaling pathway [GO:0160145] (biological process) References: PMID:35177851 Relationships: is a type of GO:0009968; is a type of regulation of cellular response to stress [GO:0080135]; negatively regulates GDF15-GFRAL signaling pathway [GO:0160144] Definition: Any process that stops, prevents or reduces the frequency, rate or extent of GDF15-GFRAL signaling pathway.